branching involved in blood vessel morphogenesis [GO:0001569] (biological process) Sources: GOC:dph Also known as: patterning of blood vessels Regulation: regulated by GO:1905553; negatively regulated by negative regulation of blood vessel branching [GO:1905554]; RO_0002213 by positive regulation of blood vessel branching [GO:1905555] Definition: The process of coordinated growth and sprouting of blood vessels giving rise to the organized vascular system. Relationships: is a type of branching morphogenesis of an epithelial tube [GO:0048754]; is part of angiogenesis [GO:0001525]